{
  "gene_symbol": "TMSB10",
  "term_label": "protein sequestering activity",
  "term_id": "GO:0140311",
  "gene_name": "Thymosin beta-10",
  "gene": "UniProtKB:P63313"
}